{
  "gene_symbol": "CCDC180",
  "term_label": "Unknown cellular component",
  "gene": "UniProtKB:Q9P1Z9",
  "gene_name": "Coiled-coil domain-containing protein 180",
  "term_id": "UNKNOWN:0003"
}